{
  "gene": "UniProtKB:Q9H568",
  "term_label": "membrane",
  "gene_symbol": "ACTL8",
  "gene_name": "Actin-like protein 8",
  "term_id": "GO:0016020"
}